{
  "gene_name": "IQ calmodulin-binding motif-containing protein 1",
  "term_id": "GO:0060271",
  "gene_symbol": "IQCB1",
  "term_label": "cilium assembly",
  "gene": "UniProtKB:Q15051"
}